{
  "term_label": "calcium-dependent cell-cell adhesion",
  "gene_name": "Cadherin-like protein 26",
  "term_id": "GO:0016339",
  "gene": "UniProtKB:Q8IXH8",
  "gene_symbol": "CDH26"
}